box C/D sno(s)RNA metabolic process [GO:0033967] (biological process) Subtypes: box C/D sno(s)RNA processing [GO:0034963] Definition: The chemical reactions and pathways involving box C/D type small nucleolar RNA. Sources: GOC:krc, GOC:mah Also known as: box C/D sRNA metabolic process, box C/D snoRNA metabolic process Relationships: is a type of GO:0016074